{
  "gene": "UniProtKB:Q68DH5",
  "gene_symbol": "LMBRD2",
  "term_label": "adrenergic receptor signaling pathway",
  "gene_name": "G-protein coupled receptor-associated protein LMBRD2",
  "term_id": "GO:0071875"
}